{
  "term_id": "GO:0008893",
  "gene_name": "Guanosine-3',5'-bis(diphosphate) 3'-pyrophosphohydrolase MESH1",
  "gene_symbol": "HDDC3",
  "gene": "UniProtKB:Q8N4P3",
  "term_label": "guanosine-3',5'-bis(diphosphate) 3'-diphosphatase activity"
}